{
  "gene_symbol": "SLC17A8",
  "term_label": "synaptic vesicle membrane",
  "gene_name": "Vesicular glutamate transporter 3",
  "gene": "UniProtKB:Q8NDX2",
  "term_id": "GO:0030672"
}